{
  "gene_symbol": "SLC35G2",
  "gene": "UniProtKB:Q8TBE7",
  "term_id": "GO:0005886",
  "gene_name": "Solute carrier family 35 member G2",
  "term_label": "plasma membrane"
}